{
  "term_id": "GO:0016887",
  "gene_name": "Kinesin heavy chain isoform 5A",
  "gene_symbol": "KIF5A",
  "term_label": "ATP hydrolysis activity",
  "gene": "UniProtKB:Q12840"
}